{
  "gene_symbol": "FANCD2OS",
  "gene": "UniProtKB:Q96PS1",
  "term_label": "Unknown cellular component",
  "term_id": "UNKNOWN:0003",
  "gene_name": "FANCD2 opposite strand protein"
}